{
  "gene_symbol": "ARMH2",
  "gene_name": "Armadillo-like helical domain-containing protein 2",
  "term_id": "UNKNOWN:0001",
  "term_label": "Unknown molecular function",
  "gene": "UniProtKB:H3BNL8"
}